{
  "gene_symbol": "PUM2",
  "term_id": "GO:0005829",
  "gene": "UniProtKB:Q8TB72",
  "term_label": "cytosol",
  "gene_name": "Pumilio homolog 2"
}